{
  "gene": "UniProtKB:Q96F81",
  "gene_symbol": "DISP1",
  "gene_name": "Protein dispatched homolog 1",
  "term_label": "membrane",
  "term_id": "GO:0016020"
}